{
  "term_id": "GO:0005513",
  "gene_name": "Extracellular calcium-sensing receptor",
  "term_label": "detection of calcium ion",
  "gene": "UniProtKB:P41180",
  "gene_symbol": "CASR"
}